{
  "term_label": "Unknown biological process",
  "term_id": "UNKNOWN:0002",
  "gene": "UniProtKB:A0A2U3TZM8",
  "gene_name": "Uncharacterized protein",
  "gene_symbol": "LOC112694756"
}